tetrahydroxybenzophenone synthase activity [GO:0047181] (molecular function) Sources: EC:2.3.1.151, MetaCyc:2.3.1.151-RXN Also known as: malonyl-CoA:3-hydroxybenzoyl-CoA malonyltransferase activity Relationships: is a type of GO:0016747 Definition: Catalysis of the reaction: 3-hydroxybenzoyl-CoA + 3 malonyl-CoA = 3 CO2 + 2,3',4,6-tetrahydroxybenzophenone + 4 coenzyme A.